{
  "gene": "UniProtKB:Q76B58",
  "gene_symbol": "BRINP3",
  "term_label": "Unknown molecular function",
  "gene_name": "BMP_retinoic acid-inducible neural-specific protein 3",
  "term_id": "UNKNOWN:0001"
}